{
  "gene": "UniProtKB:P0DV75",
  "term_label": "Unknown cellular component",
  "gene_name": "Protein FAM90A18",
  "term_id": "UNKNOWN:0003",
  "gene_symbol": "FAM90A18"
}